regulation of homoserine biosynthetic process [GO:1901710] (biological process) Also known as: regulation of homoserine anabolism, regulation of homoserine biosynthesis, regulation of homoserine formation, regulation of homoserine synthesis Relationships: is a type of regulation of small molecule metabolic process [GO:0062012]; is a type of regulation of amino acid biosynthetic process [GO:2000282]; regulates GO:0009090 Subtypes: negative regulation of homoserine biosynthetic process [GO:1901711], positive regulation of homoserine biosynthetic process [GO:1901712] Definition: Any process that modulates the frequency, rate or extent of homoserine biosynthetic process. Sources: GOC:TermGenie